{
  "gene": "UniProtKB:Q9ULW6",
  "term_label": "chromatin binding",
  "term_id": "GO:0003682",
  "gene_name": "Nucleosome assembly protein 1-like 2",
  "gene_symbol": "NAP1L2"
}